{
  "gene": "UniProtKB:Q5HYK9",
  "gene_symbol": "ZNF667",
  "gene_name": "Zinc finger protein 667",
  "term_id": "GO:0000978",
  "term_label": "RNA polymerase II cis-regulatory region sequence-specific DNA binding"
}